globoside biosynthetic process [GO:0001576] (biological process) Definition: The chemical reactions and pathways resulting in the formation of gobliosides that begins with the synthesis of a tetrasaccharide core GalNAc-beta-1,3-Gal-alpha-1,4-Gal-beta-1,4-Glc-ceramide. This core can be further elongated with the sequential addition of various carbohydrate units. References: PMID:35536927 Also known as: globo-series glycosphingolipid biosynthesis, globoside anabolism, globoside biosynthesis, globoside formation, globoside synthesis Relationships: is a type of globoside metabolic process [GO:0001575]; is a type of glycosphingolipid biosynthetic process [GO:0006688]